protein-DNA-RNA complex disassembly [GO:0001117] (biological process) Definition: The disaggregation of a protein-DNA-RNA complex into its constituent components. Subtypes: transcription ternary complex disassembly [GO:0001118] Sources: GOC:txnOH Relationships: is a type of GO:0001115; is a type of protein-containing complex disassembly [GO:0032984]